positive regulation of glutamate receptor signaling pathway [GO:1900451] (BP) Relationships: is a type of GO:0009967; is a type of regulation of glutamate receptor signaling pathway [GO:1900449]; positively regulates glutamate receptor signaling pathway [GO:0007215] Definition: Any process that activates or increases the frequency, rate or extent of glutamate receptor signaling pathway. Also known as: activation of glutamate signaling pathway, activation of glutamate signalling pathway, positive regulation of glutamate signaling pathway, positive regulation of glutamate signalling pathway, up regulation of glutamate receptor signaling pathway, up regulation of glutamate signaling pathway, up regulation of glutamate signalling pathway, up-regulation of glutamate receptor signaling pathway, up-regulation of glutamate signaling pathway, up-regulation of glutamate signalling pathway, upregulation of glutamate receptor signaling pathway, upregulation of glutamate signaling pathway, upregulation of glutamate signalling pathway, activation of glutamate receptor signaling pathway Sources: GOC:BHF, GOC:TermGenie